{
  "term_id": "UNKNOWN:0002",
  "gene_symbol": "FAM163B",
  "gene_name": "Protein FAM163B",
  "gene": "UniProtKB:P0C2L3",
  "term_label": "Unknown biological process"
}